D-amino-acid oxidase activity [GO:0003884] (molecular function) Subtypes: GO:0008445, D-glutamate(D-aspartate) oxidase activity [GO:0047819], D-glutamate oxidase activity [GO:0047821] Definition: Catalysis of the reaction: a D-alpha-amino acid + H2O + O2 = a 2-oxocarboxylate + H2O2 + NH4+. Relationships: is a type of GO:0008131 Also known as: D-amino-acid:oxygen oxidoreductase (deaminating), L-amino acid:O2 oxidoreductase activity, new yellow enzyme Sources: RHEA:21816